lipoteichoic acid catabolic process [GO:0070396] (biological process) Definition: The chemical reactions and pathways resulting in the breakdown of lipoteichoic acid, which is a major component of the cell wall of gram-positive bacteria and typically consists of a chain of glycerol-phosphate repeating units linked to a glycolipid anchor. References: PMID:14665680 Sources: GOC:add Also known as: lipoteichoic acid breakdown, lipoteichoic acid catabolism, lipoteichoic acid degradation Relationships: is_a teichoic acid catabolic process [GO:0070393]